proline transmembrane transport [GO:0035524] (biological process) Subtypes: GO:1904555, proline import across plasma membrane [GO:1905647] Definition: The directed movement of proline, pyrrolidine-2-carboxylic acid, across a membrane by means of some agent such as a transporter or pore. Sources: GOC:vw Also known as: proline membrane transport Note: Note that this term is not intended for use in annotating lateral movement within membranes. Relationships: is a type of GO:0003333; is a type of GO:0071705; is a type of carboxylic acid transmembrane transport [GO:1905039]